{
  "gene": "UniProtKB:Q04656",
  "term_id": "GO:0005886",
  "term_label": "plasma membrane",
  "gene_name": "Copper-transporting ATPase 1",
  "gene_symbol": "ATP7A"
}